oocyte development [GO:0048599] (biological process) Relationships: is a type of germ cell development [GO:0007281]; is part of GO:0009994 Sources: GOC:go_curators Definition: The process whose specific outcome is the progression of an oocyte over time, from initial commitment of the cell to its specific fate, to the fully functional differentiated cell. Regulation: regulated by regulation of oocyte development [GO:0060281]; positively regulated by GO:0060282; negatively regulated by negative regulation of oocyte development [GO:0060283]